{
  "gene_symbol": "SLC41A2",
  "gene": "UniProtKB:Q96JW4",
  "gene_name": "Solute carrier family 41 member 2",
  "term_label": "Unknown molecular function",
  "term_id": "UNKNOWN:0001"
}